{
  "term_label": "cell surface receptor signaling pathway",
  "gene_name": "T cell receptor beta chain MC.7.G5",
  "gene_symbol": "TRB",
  "gene": "UniProtKB:P0DTU4",
  "term_id": "GO:0007166"
}